{
  "gene": "UniProtKB:Q5VV52",
  "gene_name": "Zinc finger protein 691",
  "gene_symbol": "ZNF691",
  "term_id": "GO:0003700",
  "term_label": "DNA-binding transcription factor activity"
}